{
  "gene_symbol": "CD19",
  "term_id": "GO:0009897",
  "gene_name": "B-lymphocyte antigen CD19",
  "gene": "UniProtKB:P15391",
  "term_label": "external side of plasma membrane"
}